type III interferon receptor activity [GO:0034348] (molecular function) Definition: Combining with a type III interferon and transmitting the signal from one side of the membrane to the other to initiate a change in cell activity. Interferon lambda is the only member of the type III interferon found so far. References: PMID:15546383, PMID:16734557 Sources: GOC:add, GOC:signaling, ISBN:0126896631 Also known as: interferon-lambda receptor activity Note: Note that IL-28A, IL-28B, and IL-29 are types of interferon-lambda. Relationships: is a type of GO:0004904; is part of type III interferon-mediated signaling pathway [GO:0038196]; has part type III interferon binding [GO:0034347]